hydroperoxy icosatetraenoate isomerase activity [GO:0106255] (molecular function) Definition: A hydroperoxy icosatetraenoate = a hydroxy epoxy icosatrienoate. Relationships: is a type of intramolecular hydroxytransferase activity [GO:0050486] References: PMID:12881489 Sources: RHEA:55560